positive regulation of compound eye pigmentation [GO:0048078] (biological process) Definition: Any process that activates or increases the frequency, rate or extent of establishment of a pattern of pigment in the compound eye. Sources: GOC:jid Also known as: activation of eye pigmentation, positive regulation of eye pigmentation, stimulation of eye pigmentation, up regulation of eye pigmentation, up-regulation of eye pigmentation, upregulation of eye pigmentation Relationships: is a type of GO:0048075; is a type of regulation of compound eye pigmentation [GO:0048076]; positively regulates GO:0048072